{
  "term_label": "cortical cytoskeleton organization",
  "gene_symbol": "RAC1",
  "gene": "UniProtKB:P63000",
  "gene_name": "Ras-related C3 botulinum toxin substrate 1",
  "term_id": "GO:0030865"
}